cellular respiration [GO:0045333] (biological process) Relationships: is_a energy derivation by oxidation of organic compounds [GO:0015980] Regulation: regulated by regulation of cellular respiration [GO:0043457]; negatively regulated by GO:1901856; positively regulated by GO:1901857 Sources: GOC:das, ISBN:0140513590, ISBN:0198506732 Also known as: respiration, oxidative metabolic process, oxidative metabolism Subtypes: GO:0009060, anaerobic respiration [GO:0009061] Definition: The enzymatic release of energy from inorganic and organic compounds (especially carbohydrates and fats) which either requires oxygen (aerobic respiration) or does not (anaerobic respiration).